{
  "gene_name": "Embigin",
  "gene_symbol": "EMB",
  "term_label": "homophilic cell-cell adhesion",
  "term_id": "GO:0007156",
  "gene": "UniProtKB:Q6PCB8"
}